{
  "gene_symbol": "HK3",
  "term_label": "fructokinase activity",
  "term_id": "GO:0008865",
  "gene_name": "Hexokinase-3",
  "gene": "UniProtKB:P52790"
}